{
  "gene": "UniProtKB:Q92979",
  "term_label": "small-subunit processome",
  "gene_name": "Ribosomal RNA small subunit methyltransferase NEP1",
  "term_id": "GO:0032040",
  "gene_symbol": "EMG1"
}